{
  "term_label": "ubiquitin-dependent protein catabolic process",
  "term_id": "GO:0006511",
  "gene_symbol": "CUL7",
  "gene": "UniProtKB:Q14999",
  "gene_name": "Cullin-7"
}